{
  "gene": "UniProtKB:O95363",
  "term_label": "phenylalanyl-tRNA aminoacylation",
  "term_id": "GO:0006432",
  "gene_name": "Phenylalanine--tRNA ligase, mitochondrial",
  "gene_symbol": "FARS2"
}